{
  "gene": "UniProtKB:A6NDN8",
  "gene_symbol": "A6NDN8",
  "term_label": "Unknown cellular component",
  "gene_name": "Putative ubiquitin-like protein FUBI-like protein ENSP00000310146",
  "term_id": "UNKNOWN:0003"
}